negative phototaxis [GO:0046957] (biological process) Definition: The directed movement of a cell or organism away from a source of light. Relationships: is a type of phototaxis [GO:0042331]; is_a negative energy taxis [GO:0052129] Sources: GOC:ai Also known as: negative phototactic behavior, negative phototactic behaviour, negative taxis in response to light